{
  "gene_symbol": "NAA50",
  "gene_name": "N-alpha-acetyltransferase 50",
  "gene": "UniProtKB:Q9GZZ1",
  "term_id": "GO:0007064",
  "term_label": "mitotic sister chromatid cohesion"
}